{
  "gene": "UniProtKB:Q5T7M9",
  "term_label": "Unknown cellular component",
  "gene_name": "Divergent protein kinase domain 1A",
  "gene_symbol": "DIPK1A",
  "term_id": "UNKNOWN:0003"
}